vascular associated smooth muscle cell migration [GO:1904738] (BP) Also known as: vascular smooth muscle cell migration References: PMID:20693317 Sources: GOC:BHF, GOC:BHF_miRNA, GOC:TermGenie, GOC:rph, GO_REF:0000091 Definition: The orderly movement of a vascular associated smooth muscle cell from one site to another. Relationships: is a type of smooth muscle cell migration [GO:0014909] Regulation: regulated by GO:1904752; RO_0002212 by GO:1904753; positively regulated by positive regulation of vascular associated smooth muscle cell migration [GO:1904754]